tendon cell differentiation [GO:0035990] (biological process) Relationships: is a type of cell differentiation [GO:0030154]; BFO_0000050 tendon formation [GO:0035992] Also known as: muscle attachment cell differentiation, tenocyte differentiation Regulation: regulated by regulation of tendon cell differentiation [GO:2001049]; negatively regulated by negative regulation of tendon cell differentiation [GO:2001050]; positively regulated by positive regulation of tendon cell differentiation [GO:2001051] Definition: The process in which a relatively unspecialized cell acquires the specialized features of a tendon cell. Tendon cell are elongated fibrocytes in which the cytoplasm is stretched between the collagen fibres of the tendon. Tendon cells have a central cell nucleus with a prominent nucleolus, a well-developed rough endoplasmic reticulum, and are responsible for synthesis and turnover of tendon fibres and ground substance. References: PMID:21412429 Sources: CL:0000388, GOC:yaf